{
  "gene_symbol": "MT-ND5",
  "term_label": "respiratory chain complex I",
  "term_id": "GO:0045271",
  "gene_name": "NADH-ubiquinone oxidoreductase chain 5",
  "gene": "UniProtKB:P03915"
}